{
  "gene_symbol": "IFNA1",
  "gene_name": "Interferon alpha-1_13",
  "gene": "UniProtKB:P01562",
  "term_id": "GO:0006959",
  "term_label": "humoral immune response"
}